epithelial-mesenchymal signaling involved in prostate gland development [GO:0060738] (biological process) Relationships: is a type of GO:0060684; is part of prostate gland development [GO:0030850] Also known as: epithelial-mesenchymal signalling involved in prostate gland development Sources: GOC:dph Definition: Any process that results in the transfer of information from an epithelial cell to a mesenchymal cell where it is interpreted and contributes to the progression of the prostate gland over time.